microtubule polymerization based movement [GO:0099098] (biological process) Relationships: is a type of microtubule-based movement [GO:0007018]; has part microtubule polymerization [GO:0046785] Sources: GOC:cjm, ISBN:0815316194 Definition: The movement of a cellular component as a result of microtubule polymerization. Subtypes: GO:0034640, nuclear migration by microtubule mediated pushing forces [GO:0098863]